{
  "gene_name": "Zinc finger protein 732",
  "term_label": "DNA-binding transcription factor activity, RNA polymerase II-specific",
  "gene": "UniProtKB:B4DXR9",
  "gene_symbol": "ZNF732",
  "term_id": "GO:0000981"
}